{
  "gene_symbol": "IGLV8-61",
  "term_label": "immune response",
  "gene": "UniProtKB:A0A075B6I0",
  "gene_name": "Immunoglobulin lambda variable 8-61",
  "term_id": "GO:0006955"
}